{
  "gene_name": "Proline rich transmembrane protein 1B",
  "gene_symbol": "PRRT1B",
  "term_id": "UNKNOWN:0001",
  "gene": "UniProtKB:A0A1B0GWB2",
  "term_label": "Unknown molecular function"
}